{
  "term_label": "stress granule assembly",
  "term_id": "GO:0034063",
  "gene": "UniProtKB:Q13283",
  "gene_name": "Ras GTPase-activating protein-binding protein 1",
  "gene_symbol": "G3BP1"
}